{
  "gene_name": "Potassium voltage-gated channel subfamily G member 3",
  "gene": "UniProtKB:Q8TAE7",
  "term_label": "action potential",
  "term_id": "GO:0001508",
  "gene_symbol": "KCNG3"
}